{
  "term_id": "GO:0001730",
  "gene": "UniProtKB:Q9Y6K5",
  "gene_name": "2'-5'-oligoadenylate synthase 3",
  "term_label": "2'-5'-oligoadenylate synthetase activity",
  "gene_symbol": "OAS3"
}